vascular associated smooth muscle contraction [GO:0014829] (biological process) Definition: A process, occurring in the vascular tissue, whereby actin/myosin complex activity generates force through ATP hydrolysis resulting in a change in smooth muscle geometry. This process is always coupled to chemo-mechanical energy conversion. Sources: GOC:mtg_muscle, MA:0002718 Also known as: vascular smooth muscle contraction Relationships: is a type of smooth muscle contraction [GO:0006939]; is a type of vasoconstriction [GO:0042310] Subtypes: artery smooth muscle contraction [GO:0014824], vein smooth muscle contraction [GO:0014826] Regulation: regulated by regulation of vascular associated smooth muscle contraction [GO:0003056]; negatively regulated by GO:1904694; positively regulated by positive regulation of vascular associated smooth muscle contraction [GO:1904695]